1,3-beta-D-glucan synthase complex [GO:0000148] (cellular component) References: PMID:7983071 Also known as: (1->3)-beta-glucan synthase complex, 1,3-beta-glucan synthase complex Relationships: is a type of transferase complex [GO:1990234] Definition: A protein complex that catalyzes the transfer of a glucose group from UDP-glucose to a (1->3)-beta-D-glucan chain.